{
  "gene_symbol": "GTPBP4",
  "term_label": "GTPase activity",
  "gene_name": "GTP-binding protein 4",
  "gene": "UniProtKB:Q9BZE4",
  "term_id": "GO:0003924"
}